negative regulation of pigment cell differentiation [GO:0050941] (biological process) Definition: Any process that stops, prevents, or reduces the frequency, rate or extent of pigment cell differentiation. Sources: GOC:ai Also known as: down regulation of pigment cell differentiation, down-regulation of pigment cell differentiation, downregulation of pigment cell differentiation, inhibition of pigment cell differentiation Relationships: is a type of GO:0045596; is a type of GO:0048086; is a type of regulation of pigment cell differentiation [GO:0050932]; negatively regulates GO:0050931 Subtypes: negative regulation of melanocyte differentiation [GO:0045635], negative regulation of leucophore differentiation [GO:0048776], negative regulation of erythrophore differentiation [GO:0048779], GO:0048782, GO:0050943, negative regulation of xanthophore differentiation [GO:0050944]